{
  "gene_symbol": "LPL",
  "term_id": "GO:0004465",
  "term_label": "lipoprotein lipase activity",
  "gene": "UniProtKB:P06858",
  "gene_name": "Lipoprotein lipase"
}